{
  "gene_name": "Cation-independent mannose-6-phosphate receptor",
  "term_id": "GO:0005886",
  "gene": "UniProtKB:P11717",
  "term_label": "plasma membrane",
  "gene_symbol": "IGF2R"
}